{
  "term_label": "Unknown molecular function",
  "gene_symbol": "CUBN",
  "gene": "UniProtKB:O60494",
  "term_id": "UNKNOWN:0001",
  "gene_name": "Cubilin"
}